{
  "term_label": "plasma membrane",
  "gene_symbol": "ADAM9",
  "gene_name": "Disintegrin and metalloproteinase domain-containing protein 9",
  "gene": "UniProtKB:Q13443",
  "term_id": "GO:0005886"
}